{
  "term_id": "UNKNOWN:0001",
  "gene_name": "Killin",
  "term_label": "Unknown molecular function",
  "gene_symbol": "KLLN",
  "gene": "UniProtKB:B2CW77"
}